{
  "gene_name": "Kynurenine 3-monooxygenase",
  "term_label": "mitochondrial outer membrane",
  "term_id": "GO:0005741",
  "gene": "UniProtKB:O15229",
  "gene_symbol": "KMO"
}